{
  "term_id": "UNKNOWN:0002",
  "gene_symbol": "CARD19",
  "gene": "UniProtKB:Q96LW7",
  "gene_name": "Caspase recruitment domain-containing protein 19",
  "term_label": "Unknown biological process"
}